{
  "gene": "UniProtKB:P78333",
  "gene_name": "Glypican-5",
  "gene_symbol": "GPC5",
  "term_label": "regulation of protein localization to membrane",
  "term_id": "GO:1905475"
}